atrazine catabolic process to cyanuric acid [GO:0019625] (biological process) Also known as: atrazine breakdown to cyanuric acid, atrazine degradation to cyanuric acid Definition: The chemical reactions and pathways resulting in the breakdown of atrazine, a triazine ring-containing herbicide, into cyanuric acid. Sources: GOC:jl Relationships: is a type of atrazine catabolic process [GO:0019381]